{
  "gene": "UniProtKB:O94933",
  "term_id": "GO:0098839",
  "term_label": "postsynaptic density membrane",
  "gene_name": "SLIT and NTRK-like protein 3",
  "gene_symbol": "SLITRK3"
}